histone reader activity [GO:0140566] (molecular function) Definition: A chromatin adaptor activity that brings together a protein and a specific form of histone, either modified by a post-translational modification, or the unmodified form. Histone readers have roles in many processes, including in centromere function or in modulating the accessibility of cis-regulatory regions to the transcription machinery. References: PMID:11498575, PMID:25688442, PMID:31082667, PMID:34726351 Also known as: epigenetic reader, histone reader Relationships: is a type of chromatin-protein adaptor activity [GO:0140463]; has part histone binding [GO:0042393]; occurs in GO:0000786 Subtypes: ubiquitin-modified histone reader activity [GO:0061649], histone H3 reader activity [GO:0140006], GO:0140008, histone H2A reader activity [GO:0140054], unmodified histone reader activity [GO:0140063], histone H2B reader activity [GO:0140071], histone H1 reader activity [GO:0140128]